{
  "gene": "UniProtKB:Q6UX15",
  "gene_name": "Layilin",
  "term_id": "GO:0005540",
  "term_label": "hyaluronic acid binding",
  "gene_symbol": "LAYN"
}